{
  "gene_symbol": "SH3RF2",
  "term_id": "GO:0046330",
  "gene_name": "E3 ubiquitin-protein ligase SH3RF2",
  "gene": "UniProtKB:Q8TEC5",
  "term_label": "positive regulation of JNK cascade"
}